{
  "term_id": "GO:0038023",
  "term_label": "signaling receptor activity",
  "gene": "UniProtKB:Q5T2D2",
  "gene_symbol": "TREML2",
  "gene_name": "Trem-like transcript 2 protein"
}